{
  "term_label": "Unknown molecular function",
  "term_id": "UNKNOWN:0001",
  "gene_symbol": "MREG",
  "gene_name": "Melanoregulin",
  "gene": "UniProtKB:Q8N565"
}